vascular associated smooth muscle cell fate specification [GO:0097082] (biological process) Also known as: vascular smooth muscle cell fate specification Sources: GOC:BHF Relationships: is_a muscle cell fate specification [GO:0042694]; BFO_0000050 GO:0097081 Definition: The process in which a cell becomes capable of differentiating autonomously into a vascular smooth muscle cell in an environment that is neutral with respect to the developmental pathway. Upon specification, the cell fate can be reversed. A vascular smooth muscle cell is a non-striated, elongated, spindle-shaped cell found lining the blood vessels.